{
  "term_label": "phosphatidylinositol 3-kinase binding",
  "gene_symbol": "BECN1",
  "term_id": "GO:0043548",
  "gene_name": "Beclin-1",
  "gene": "UniProtKB:Q14457"
}